{
  "gene": "UniProtKB:P34896",
  "gene_symbol": "SHMT1",
  "gene_name": "Serine hydroxymethyltransferase, cytosolic",
  "term_id": "GO:0004372",
  "term_label": "glycine hydroxymethyltransferase activity"
}